{
  "gene": "UniProtKB:Q06418",
  "term_label": "phagocytosis",
  "gene_name": "Tyrosine-protein kinase receptor TYRO3",
  "term_id": "GO:0006909",
  "gene_symbol": "TYRO3"
}